{
  "gene": "UniProtKB:Q9NTZ6",
  "term_id": "GO:0003723",
  "gene_symbol": "RBM12",
  "gene_name": "RNA-binding protein 12",
  "term_label": "RNA binding"
}